type 1 member 1 taste receptor binding [GO:0031884] (molecular function) Sources: GOC:mah, GOC:nln Relationships: is a type of taste receptor binding [GO:0031883] Definition: Binding to a type 1 member 1 taste receptor. Also known as: type 1 member 1 taste receptor ligand